{
  "gene": "UniProtKB:Q8NCG5",
  "gene_name": "Carbohydrate sulfotransferase 4",
  "term_id": "GO:0001517",
  "term_label": "N-acetylglucosamine 6-O-sulfotransferase activity",
  "gene_symbol": "CHST4"
}